protein-cysteine S-palmitoyltransferase complex [GO:1905961] (cellular component) References: PMID:20851885 Sources: GOC:TermGenie, GOC:bhm, GO_REF:0000088 Relationships: is a type of palmitoyltransferase complex [GO:0002178] Definition: A protein complex which is capable of protein-cysteine S-palmitoyltransferase activity. Also known as: Palmitoyltransferase ERF2-SHR5 complex, Palmitoyltransferase ERF2/SHR5 complex Note: An example of this is ERF2 in Saccharomyces cerevisiae (Q06551) in PMID:20851885 (inferred from direct assay)